{
  "term_id": "GO:0030055",
  "term_label": "cell-substrate junction",
  "gene": "UniProtKB:Q15124",
  "gene_symbol": "PGM5",
  "gene_name": "Phosphoglucomutase-like protein 5"
}